{
  "gene": "UniProtKB:Q8NBB2",
  "gene_name": "Putative uncharacterized protein ST20-AS1",
  "gene_symbol": "ST20-AS1",
  "term_label": "Unknown biological process",
  "term_id": "UNKNOWN:0002"
}